{
  "term_id": "GO:0016887",
  "gene_symbol": "PEX6",
  "gene_name": "Peroxisomal ATPase PEX6",
  "term_label": "ATP hydrolysis activity",
  "gene": "UniProtKB:Q13608"
}